{
  "term_label": "Unknown molecular function",
  "gene": "UniProtKB:Q9BZQ2",
  "gene_symbol": "SHCBP1L",
  "gene_name": "Testicular spindle-associated protein SHCBP1L",
  "term_id": "UNKNOWN:0001"
}